{
  "term_label": "Unknown molecular function",
  "term_id": "UNKNOWN:0001",
  "gene": "UniProtKB:Q15049",
  "gene_name": "Membrane protein MLC1",
  "gene_symbol": "MLC1"
}